{
  "gene_symbol": "TRUB2",
  "term_id": "GO:1990481",
  "term_label": "mRNA pseudouridine synthesis",
  "gene": "UniProtKB:O95900",
  "gene_name": "Pseudouridylate synthase TRUB2, mitochondrial"
}